immunoglobulin V(D)J recombination [GO:0033152] (biological process) Subtypes: immunoglobulin heavy chain V-D-J recombination [GO:0071707], immunoglobulin light chain V-J recombination [GO:0071708] Definition: The process in which immunoglobulin gene segments are recombined within a single locus utilizing the conserved heptamer and nonomer recombination signal sequences (RSS). For immunoglobulin heavy chains V, D, and J gene segments are joined, and for immunoglobulin light chains V and J gene segments are joined. Relationships: is a type of somatic recombination of immunoglobulin gene segments [GO:0016447]; is a type of V(D)J recombination [GO:0033151] Also known as: immunoglobulin V(D)J joining, immunoglobulin V-D-J joining, immunoglobulin V-D-J recombination, immunoglobulin V-J joining, immunoglobulin V-J recombination Sources: GOC:add, ISBN:0781735149